positive regulation of CREB transcription factor activity [GO:0032793] (biological process) Definition: Any process that activates or increases the frequency, rate or extent of activity of the transcription factor CREB. Also known as: activation of CREB, activation of CREB transcription factor, CREB activator Relationships: is a type of positive regulation of DNA-binding transcription factor activity [GO:0051091] Sources: GOC:dph, GOC:ecd, GOC:tb